pentose transmembrane transporter activity [GO:0015146] (molecular function) Definition: Enables the transfer of a pentose sugar from one side of a membrane to the other. Pentose is a monosaccharide with 5 carbon atoms. Sources: GOC:ai, GOC:mtg_transport, ISBN:0815340729 Relationships: is a type of monosaccharide transmembrane transporter activity [GO:0015145]; is part of pentose transmembrane transport [GO:0015750] Subtypes: D-xylose transmembrane transporter activity [GO:0015148], GO:0015591, GO:0042900